{
  "gene_name": "Kelch-like ECH-associated protein 1",
  "gene": "UniProtKB:Q14145",
  "term_id": "GO:0005737",
  "term_label": "cytoplasm",
  "gene_symbol": "KEAP1"
}